glomerular parietal epithelial cell differentiation [GO:0072139] (biological process) Definition: The process in which a relatively unspecialized cell acquires specialized features of a glomerular parietal epithelial cell. Glomerular parietal epithelial cells are specialized epithelial cells that form tight junctions as a barrier to protein transport. Sources: GOC:mtg_kidney_jan10 Relationships: is a type of GO:0072311 Subtypes: mesonephric glomerular parietal epithelial cell differentiation [GO:0061253], metanephric glomerular parietal epithelial cell differentiation [GO:0072245]